{
  "gene": "UniProtKB:O43448",
  "gene_symbol": "KCNAB3",
  "term_id": "GO:0008076",
  "term_label": "voltage-gated potassium channel complex",
  "gene_name": "Voltage-gated potassium channel subunit beta-3"
}